{
  "gene_name": "ATP-dependent RNA helicase DDX50",
  "gene_symbol": "DDX50",
  "gene": "UniProtKB:Q9BQ39",
  "term_label": "Unknown biological process",
  "term_id": "UNKNOWN:0002"
}